{
  "gene_symbol": "IGLV2-33",
  "term_id": "GO:0006955",
  "term_label": "immune response",
  "gene": "UniProtKB:A0A075B6J2",
  "gene_name": "Probable non-functional immunoglobulin lambda variable 2-33"
}